{
  "gene": "UniProtKB:Q59GN2",
  "term_id": "GO:0022625",
  "gene_symbol": "RPL39P5",
  "gene_name": "Putative ribosomal protein eL39-like 5",
  "term_label": "cytosolic large ribosomal subunit"
}